{
  "gene_symbol": "HSD11B1",
  "gene_name": "11-beta-hydroxysteroid dehydrogenase 1",
  "gene": "UniProtKB:P28845",
  "term_label": "endoplasmic reticulum membrane",
  "term_id": "GO:0005789"
}